{
  "gene_symbol": "RRP7A",
  "gene": "UniProtKB:Q9Y3A4",
  "gene_name": "Ribosomal RNA-processing protein 7 homolog A",
  "term_id": "GO:0034456",
  "term_label": "UTP-C complex"
}